{
  "gene": "UniProtKB:Q8IYI8",
  "term_id": "GO:0006357",
  "term_label": "regulation of transcription by RNA polymerase II",
  "gene_name": "Zinc finger protein 440",
  "gene_symbol": "ZNF440"
}